D-lactate dehydrogenase (quinone) activity [GO:0102029] (molecular function) Relationships: is a type of D-lactate dehydrogenase activity [GO:0047809]; is a type of GO:1990464 Definition: Catalysis of the reaction: (R)-lactate + an ubiquinone = pyruvate + an ubiquinol. Also known as: D-lactate dehydrogenase activity References: PMID:10944213, PMID:4575624 Sources: RHEA:51468